{
  "gene": "UniProtKB:Q16611",
  "term_label": "channel activity",
  "term_id": "GO:0015267",
  "gene_symbol": "BAK1",
  "gene_name": "Bcl-2 homologous antagonist_killer"
}